{
  "gene_name": "Creatine kinase B-type",
  "gene_symbol": "CKB",
  "gene": "UniProtKB:P12277",
  "term_id": "GO:0004111",
  "term_label": "creatine kinase activity"
}